{
  "term_label": "endoplasmic reticulum to Golgi vesicle-mediated transport",
  "gene_symbol": "RINT1",
  "gene_name": "RAD50-interacting protein 1",
  "term_id": "GO:0006888",
  "gene": "UniProtKB:Q6NUQ1"
}